{
  "term_label": "regulation of transcription by RNA polymerase II",
  "gene": "UniProtKB:O95125",
  "term_id": "GO:0006357",
  "gene_name": "Zinc finger protein 202",
  "gene_symbol": "ZNF202"
}